positive regulation of transcription by RNA polymerase II [GO:0045944] (BP) Subtypes: carbon catabolite activation of transcription from RNA polymerase II promoter [GO:0000436], positive regulation of transcription of Notch receptor target [GO:0007221], positive regulation of transcription elongation by RNA polymerase II [GO:0032968], positive regulation of transcription initiation by RNA polymerase II [GO:0060261], positive regulation of ribosomal protein gene transcription by RNA polymerase II [GO:0060963], positive regulation of pseudohyphal growth by positive regulation of transcription from RNA polymerase II promoter [GO:1900461], positive regulation of snRNA transcription by RNA polymerase II [GO:1905382] Definition: Any process that activates or increases the frequency, rate or extent of transcription from an RNA polymerase II promoter. Sources: GOC:go_curators, GOC:txnOH Also known as: activation of transcription from RNA polymerase II promoter, positive regulation of transcription from Pol II promoter, positive regulation of transcription from RNA polymerase II promoter, stimulation of transcription from RNA polymerase II promoter, up regulation of transcription from RNA polymerase II promoter, up-regulation of transcription from RNA polymerase II promoter, upregulation of transcription from RNA polymerase II promoter, stimulation of global transcription from RNA polymerase II promoter, activation of global transcription from RNA polymerase II promoter, positive regulation of gene-specific transcription from RNA polymerase II promoter, positive regulation of global transcription from Pol II promoter, positive regulation of transcription from RNA polymerase II promoter, global, up regulation of global transcription from RNA polymerase II promoter, up-regulation of global transcription from RNA polymerase II promoter, upregulation of global transcription from RNA polymerase II promoter Relationships: is a type of regulation of transcription by RNA polymerase II [GO:0006357]; is a type of positive regulation of DNA-templated transcription [GO:0045893]; positively regulates transcription by RNA polymerase II [GO:0006366]